{
  "term_id": "UNKNOWN:0003",
  "term_label": "Unknown cellular component",
  "gene_name": "WW domain-binding protein 1",
  "gene_symbol": "WBP1",
  "gene": "UniProtKB:Q96G27"
}